defense response to Gram-positive bacterium [GO:0050830] (biological process) Definition: Reactions triggered in response to the presence of a Gram-positive bacterium that act to protect the cell or organism. Relationships: is a type of GO:0042742 Also known as: defence response to Gram-positive bacteria, defence response to Gram-positive bacterium, defense response to Gram-positive bacteria, Gram-positive antibacterial peptide activity Sources: GOC:ai